negative regulation of membrane invagination [GO:1905154] (biological process) Also known as: down regulation of membrane invagination, down-regulation of membrane invagination, downregulation of membrane invagination, inhibition of membrane invagination Subtypes: GO:0060101 Relationships: is a type of negative regulation of cellular component organization [GO:0051129]; is a type of GO:1905153; negatively regulates membrane invagination [GO:0010324] References: PMID:26589353 Sources: GOC:PARL, GOC:TermGenie, GOC:bf, GO_REF:0000058 Definition: Any process that stops, prevents or reduces the frequency, rate or extent of membrane invagination.